deoxyuridine 2'-dioxygenase activity [GO:0047080] (molecular function) Also known as: pyrimidine deoxyribonucleoside 2'-hydroxylase activity, pyrimidine-deoxynucleoside 2'-dioxygenase activity, pyrimidine-deoxynucleoside,2-oxoglutarate 2'-dioxygenase activity, thymidine 2'-dioxygenase activity, 2'-deoxyuridine,2-oxoglutarate:oxygen oxidoreductase (2'-hydroxylating), deoxyuridine 2'-hydroxylase activity, thymidine 2'-hydroxylase activity, thymidine 2-oxoglutarate dioxygenase activity, thymidine dioxygenase activity Definition: Catalysis of the reaction: 2'-deoxyuridine + 2-oxoglutarate + O2 = CO2 + succinate + uridine. Sources: EC:1.14.11.3, RHEA:21076 Relationships: is a type of GO:0016706